clathrin-sculpted gamma-aminobutyric acid transport vesicle membrane [GO:0061202] (cellular component) Relationships: is a type of clathrin-coated vesicle membrane [GO:0030665]; is part of clathrin-sculpted gamma-aminobutyric acid transport vesicle [GO:0061200] Sources: GOC:dph Also known as: clathrin sculpted GABA transport vesicle membrane, clathrin sculpted gamma-aminobutyric acid transport vesicle membrane Definition: The lipid bilayer surrounding a clathrin-sculpted gamma-aminobutyric acid transport vesicle.